{
  "term_id": "GO:0045765",
  "term_label": "regulation of angiogenesis",
  "gene_symbol": "BMPER",
  "gene_name": "BMP-binding endothelial regulator protein",
  "gene": "UniProtKB:Q8N8U9"
}